{
  "gene_name": "Nuclear pore complex protein Nup88",
  "term_id": "GO:0000056",
  "gene": "UniProtKB:Q99567",
  "gene_symbol": "NUP88",
  "term_label": "ribosomal small subunit export from nucleus"
}